{
  "gene_symbol": "KIF21B",
  "gene_name": "Kinesin-like protein KIF21B",
  "term_id": "GO:0005874",
  "gene": "UniProtKB:O75037",
  "term_label": "microtubule"
}